{
  "gene_symbol": "CACNG8",
  "term_label": "voltage-gated calcium channel activity",
  "gene_name": "Voltage-dependent calcium channel gamma-8 subunit",
  "gene": "UniProtKB:Q8WXS5",
  "term_id": "GO:0005245"
}